{
  "gene": "UniProtKB:Q7Z3G6",
  "gene_symbol": "PRICKLE2",
  "term_id": "UNKNOWN:0003",
  "gene_name": "Prickle-like protein 2",
  "term_label": "Unknown cellular component"
}